{
  "term_id": "GO:0034472",
  "gene_symbol": "INTS9",
  "gene_name": "Integrator complex subunit 9",
  "gene": "UniProtKB:Q9NV88",
  "term_label": "snRNA 3'-end processing"
}